{
  "gene": "UniProtKB:O14656",
  "gene_name": "Torsin-1A",
  "term_id": "GO:0034504",
  "gene_symbol": "TOR1A",
  "term_label": "protein localization to nucleus"
}